{
  "gene_name": "Succinate dehydrogenase [ubiquinone] cytochrome b small subunit, mitochondrial",
  "gene_symbol": "SDHD",
  "gene": "UniProtKB:O14521",
  "term_label": "mitochondrial electron transport, succinate to ubiquinone",
  "term_id": "GO:0006121"
}